{
  "term_id": "UNKNOWN:0003",
  "term_label": "Unknown cellular component",
  "gene_symbol": "UGT2B15",
  "gene": "UniProtKB:P54855",
  "gene_name": "UDP-glucuronosyltransferase 2B15"
}